{
  "gene_name": "Glucose-dependent insulinotropic receptor",
  "gene": "UniProtKB:Q8TDV5",
  "gene_symbol": "GPR119",
  "term_label": "adenylate cyclase-activating G protein-coupled receptor signaling pathway",
  "term_id": "GO:0007189"
}